{
  "gene_symbol": "CHD8",
  "gene": "UniProtKB:Q9HCK8",
  "term_id": "GO:0003677",
  "term_label": "DNA binding",
  "gene_name": "Chromodomain-helicase-DNA-binding protein 8"
}